{
  "gene_name": "Protein SCAF11",
  "term_label": "spliceosomal complex assembly",
  "gene_symbol": "SCAF11",
  "gene": "UniProtKB:Q99590",
  "term_id": "GO:0000245"
}